{
  "term_id": "GO:0009653",
  "term_label": "anatomical structure morphogenesis",
  "gene_symbol": "FOXL2",
  "gene": "UniProtKB:P58012",
  "gene_name": "Forkhead box protein L2"
}